sulochrin oxidase [(-)-bisdechlorogeodin-forming] activity [GO:0047065] (molecular function) Definition: Catalysis of the reaction: O2 + 2 sulochrin = 2 (2R)-bisdechlorogeodin + 2 H2O. Sources: EC:1.21.3.5, RHEA:22616 Also known as: sulochrin oxidase activity, sulochrin:oxygen oxidoreductase (cyclizing, (-)-specific) Relationships: is a type of GO:0046993